starch biosynthetic process [GO:0019252] (biological process) Subtypes: starch granule initiation [GO:0062052] Also known as: starch anabolism, starch biosynthesis, starch formation, starch synthesis Regulation: regulated by regulation of starch biosynthetic process [GO:0010581]; RO_0002212 by negative regulation of starch biosynthetic process [GO:7770012] Definition: The chemical reactions and pathways resulting in the formation of starch, the most important reserve polysaccharide in plants. Relationships: is a type of starch metabolic process [GO:0005982]; is a type of GO:0009250 Sources: GOC:ai